{
  "gene": "UniProtKB:Q03181",
  "gene_symbol": "PPARD",
  "term_label": "intracellular receptor signaling pathway",
  "gene_name": "Peroxisome proliferator-activated receptor delta",
  "term_id": "GO:0030522"
}